corticotrophin-releasing factor receptor activity [GO:0015056] (molecular function) Relationships: is a type of G protein-coupled receptor activity [GO:0004930]; is part of cellular response to corticotropin-releasing hormone stimulus [GO:0071376] Definition: Combining with the corticotrophin-releasing factor family of ligands, including the urocortins, to initiate a change in cell activity. References: PMID:12032352